negative regulation of epithelial cell proliferation [GO:0050680] (biological process) Subtypes: negative regulation of endothelial cell proliferation [GO:0001937], negative regulation of keratinocyte proliferation [GO:0010839], GO:0033600, negative regulation of urothelial cell proliferation [GO:0050676], negative regulation of epithelial cell proliferation involved in prostate gland development [GO:0060770], negative regulation of synoviocyte proliferation [GO:1901646], negative regulation of sebum secreting cell proliferation [GO:1904003], GO:1904055, negative regulation of granulosa cell proliferation [GO:1904196], negative regulation of thyroid gland epithelial cell proliferation [GO:1904442], GO:1904691, GO:1904698, negative regulation of hepatocyte proliferation [GO:2000346], negative regulation of epithelial cell proliferation involved in lung morphogenesis [GO:2000795], GO:2001110 Sources: GOC:ai Definition: Any process that stops, prevents or reduces the rate or extent of epithelial cell proliferation. Relationships: is a type of negative regulation of cell population proliferation [GO:0008285]; is a type of regulation of epithelial cell proliferation [GO:0050678]; negatively regulates epithelial cell proliferation [GO:0050673] Also known as: down regulation of epithelial cell proliferation, down-regulation of epithelial cell proliferation, downregulation of epithelial cell proliferation, inhibition of epithelial cell proliferation